central plaque of mitotic spindle pole body [GO:0061493] (cellular component) Sources: GOC:dph Definition: One of three laminate structures that form the mitotic spindle pole body; the inner plaque is on the nuclear face of the spindle pole body. Relationships: is a type of central plaque of spindle pole body [GO:0005823]; is part of mitotic spindle pole body [GO:0044732]